perineurial glial growth [GO:0042066] (biological process) Definition: Glial cell growth that occurs in the perineurium, a cell layer that ensheaths projections of peripheral nerves, such as motor axons. Relationships: is a type of glial cell growth [GO:0042065] References: PMID:11517334, PMID:18176560 Sources: GOC:mah